pyruvate dehydrogenase (lipoamide) phosphatase complex [GO:0045253] (cellular component) Relationships: is_a protein serine/threonine phosphatase complex [GO:0008287]; is part of cytoplasm [GO:0005737] References: PMID:9395502 Subtypes: GO:0019910, cytosol pyruvate dehydrogenase (lipoamide) phosphatase complex [GO:0045249] Definition: A complex of a regulatory and catalytic subunit that catalyzes the dephosphorylation and concomitant reactivation of the alpha subunit of the E1 component of the pyruvate dehydrogenase complex. Note: See also the cellular component term 'cytosolic pyruvate dehydrogenase complex ; GO:0045250'.